{
  "term_label": "odorant binding",
  "gene_name": "Olfactory receptor 8B12",
  "gene": "UniProtKB:Q8NGG6",
  "gene_symbol": "OR8B12",
  "term_id": "GO:0005549"
}